{
  "term_label": "protein secretion",
  "term_id": "GO:0009306",
  "gene_name": "Small vasohibin-binding protein",
  "gene": "UniProtKB:Q8N300",
  "gene_symbol": "SVBP"
}